{
  "gene_name": "Probable ribonuclease ZC3H12C",
  "gene_symbol": "ZC3H12C",
  "term_label": "nucleus",
  "term_id": "GO:0005634",
  "gene": "UniProtKB:Q9C0D7"
}